{
  "gene": "UniProtKB:Q96BD6",
  "term_id": "GO:0019005",
  "gene_name": "SPRY domain-containing SOCS box protein 1",
  "term_label": "SCF ubiquitin ligase complex",
  "gene_symbol": "SPSB1"
}